{
  "term_label": "cytoplasm",
  "term_id": "GO:0005737",
  "gene_symbol": "CYP2C18",
  "gene_name": "Cytochrome P450 2C18",
  "gene": "UniProtKB:P33260"
}